ectodermal digestive tract development [GO:0007439] (biological process) Subtypes: ectodermal digestive tract morphogenesis [GO:0048567], post-embryonic ectodermal digestive tract development [GO:0048612] Definition: The process whose specific outcome is the progression of the ectodermal digestive tract over time, from its formation to the mature structure. The ectodermal digestive tract includes those portions that are derived from ectoderm. Also known as: ectodermal gut development Relationships: is a type of tissue morphogenesis [GO:0048729]; is part of GO:0048565 Sources: GOC:curators